{
  "gene_symbol": "HERC2P3",
  "term_id": "GO:0016567",
  "gene": "UniProtKB:Q9BVR0",
  "term_label": "protein ubiquitination",
  "gene_name": "Putative HERC2-like protein 3"
}